negative regulation of response to nutrient levels [GO:0032108] (biological process) Also known as: down regulation of response to nutrient levels, down-regulation of response to nutrient levels, downregulation of response to nutrient levels, inhibition of response to nutrient levels Definition: Any process that stops, prevents, or reduces the frequency, rate or extent of a response to nutrient levels. Sources: GOC:mah Relationships: is a type of GO:0032107; is a type of negative regulation of response to stimulus [GO:0048585]; negatively regulates response to nutrient levels [GO:0031667] Subtypes: negative regulation of cellular response to nitrogen starvation [GO:0010516], GO:0031286, negative regulation of response to food [GO:0032096], negative regulation of nitrogen utilization [GO:0045847], negative regulation of sulfur utilization [GO:0045882], negative regulation of aggregation involved in sorocarp development [GO:0110014], negative regulation of cellular response to phosphate starvation [GO:0140256], negative regulation of cellular response to iron ion starvation [GO:1901967], negative regulation of cellular response to amino acid starvation [GO:1903574]